{
  "term_id": "UNKNOWN:0001",
  "term_label": "Unknown molecular function",
  "gene": "UniProtKB:Q96DN5",
  "gene_name": "TBC1 domain family member 31",
  "gene_symbol": "TBC1D31"
}